{
  "gene_symbol": "ZNF273",
  "term_label": "Unknown cellular component",
  "gene": "UniProtKB:Q14593",
  "gene_name": "Zinc finger protein 273",
  "term_id": "UNKNOWN:0003"
}